{
  "gene_symbol": "ABITRAM",
  "gene_name": "Protein Abitram",
  "gene": "UniProtKB:Q9NX38",
  "term_label": "filopodium tip",
  "term_id": "GO:0032433"
}